hydrogen biosynthetic process [GO:1902422] (biological process) Definition: The chemical reactions and pathways resulting in the formation of H2 (dihydrogen). Relationships: is a type of biosynthetic process [GO:0009058]; is a type of hydrogen metabolic process [GO:1902421] Subtypes: fermentative hydrogen production [GO:0044812], hydrogen generation via biophotolysis [GO:0044817], GO:0044835 References: PMID:20395274, PMID:20692761 Sources: GOC:TermGenie, GOC:mengo_curators Also known as: H2 biosynthesis, dihydrogen synthesis, hydrogen anabolism, hydrogen biosynthesis, hydrogen formation, hydrogen generation, hydrogen production, hydrogen synthesis, molecular hydrogen biosynthesis